3-propylmalate synthase activity [GO:0050442] (molecular function) Definition: Catalysis of the reaction: glyoxylate + H2O + pentanoyl-CoA = 3-propylmalate + CoA + H+. Sources: RHEA:14457 Also known as: 3-(n-propyl)-malate synthase activity, 3-propylmalate glyoxylate-lyase (CoA-pentanoylating) activity, N-propylmalate synthase activity, beta-n-propylmalate synthase activity, pentanoyl-CoA:glyoxylate C-pentanoyltransferase (thioester-hydrolysing, 1-carboxybutyl-forming) Relationships: is a type of GO:0046912